epinephrine uptake [GO:0051625] (biological process) Also known as: adrenaline reuptake, adrenaline uptake, epinephrine import, epinephrine reuptake Regulation: regulated by regulation of epinephrine uptake [GO:0051626]; negatively regulated by negative regulation of epinephrine uptake [GO:0051627]; positively regulated by positive regulation of epinephrine uptake [GO:0051628] Definition: The directed movement of epinephrine into a cell, typically presynaptic neurons or glial cells. Epinephrine is a hormone produced by the medulla of the adrenal glands that increases heart activity, improves the power and prolongs the action of muscles, and increases the rate and depth of breathing. It is synthesized by the methylation of norepinephrine. Sources: GOC:ai Relationships: is a type of transport [GO:0006810]